{
  "gene_symbol": "TLR5",
  "term_label": "plasma membrane",
  "term_id": "GO:0005886",
  "gene": "UniProtKB:O60602",
  "gene_name": "Toll-like receptor 5"
}